peroxisome-chloroplast membrane tethering [GO:0010381] (biological process) Relationships: is a type of organelle localization by membrane tethering [GO:0140056] Also known as: attachment of peroxisome to chloroplast Definition: The attachment of a peroxisome to a chloroplast via molecular tethers that physically bridge their respective membranes and attach them to each other. The tethering may facilitate exchange of metabolites between the organelles. References: PMID:17215364